B cell negative selection [GO:0002352] (biological process) Also known as: B lymphocyte negative selection, B-cell negative selection, B-lymphocyte negative selection Relationships: is a type of B cell selection [GO:0002339] Sources: GOC:jal Definition: Any process leading to negative selection in B cells. Mechanisms of negative selection include anergy and deletion. Subtypes: central B cell negative selection [GO:0002354], peripheral B cell negative selection [GO:0002356]